{
  "term_id": "GO:0043197",
  "gene_symbol": "LZTS3",
  "term_label": "dendritic spine",
  "gene_name": "Leucine zipper putative tumor suppressor 3",
  "gene": "UniProtKB:O60299"
}